{
  "gene_symbol": "HPGDS",
  "term_id": "UNKNOWN:0003",
  "gene": "UniProtKB:O60760",
  "term_label": "Unknown cellular component",
  "gene_name": "Hematopoietic prostaglandin D synthase"
}